{
  "gene": "UniProtKB:Q86UN6",
  "term_label": "protein kinase A regulatory subunit binding",
  "gene_symbol": "AKAP14",
  "gene_name": "A-kinase anchor protein 14",
  "term_id": "GO:0034237"
}